{
  "term_id": "GO:0005730",
  "gene_name": "Ribosome biogenesis protein BRX1 homolog",
  "term_label": "nucleolus",
  "gene": "UniProtKB:Q8TDN6",
  "gene_symbol": "BRIX1"
}